macrophage proliferation [GO:0061517] (biological process) Relationships: is a type of leukocyte proliferation [GO:0070661] Definition: The expansion of a macrophage population by cell division. Subtypes: microglial cell proliferation [GO:0061518] Regulation: regulated by regulation of macrophage proliferation [GO:0120040]; positively regulated by positive regulation of macrophage proliferation [GO:0120041]; negatively regulated by GO:0120042 References: PMID:12614284, PMID:19466391 Sources: GOC:dph